{
  "term_id": "UNKNOWN:0002",
  "gene_name": "Transmembrane and coiled-coil domain-containing protein 5B",
  "term_label": "Unknown biological process",
  "gene": "UniProtKB:A8MYB1",
  "gene_symbol": "TMCO5B"
}